viral budding from nuclear membrane [GO:0046765] (biological process) Definition: A viral budding that starts with formation of a membrane curvature in the host nuclear membrane. Also known as: nuclear membrane viral budding, virus budding from nuclear membrane, virus budding from nuclear membrane by viral capsid envelopment, nuclear membrane viral budding during viral capsid envelopment, viral budding from nuclear membrane by viral capsid envelopment, viral budding from nuclear membrane during viral capsid envelopment, virus budding from nuclear membrane during viral capsid envelopment Sources: GOC:bf, ISBN:0072370319 Relationships: is a type of GO:0046755; is part of exit of virus from host cell nucleus by nuclear egress [GO:0046802] Subtypes: GO:0046771, viral budding from outer nuclear membrane [GO:0046772]